indole glucosinolate biosynthetic process [GO:0009759] (biological process) Also known as: indole glucosinolate anabolism, indole glucosinolate biosynthesis, indole glucosinolate formation, indole glucosinolate synthesis Definition: The chemical reactions and pathways resulting in the formation of indole glucosinolates, sulfur-containing compounds that have a common structure linked to an R group derived from tryptophan. Relationships: is a type of glucosinolate biosynthetic process [GO:0019761]; is a type of indole glucosinolate metabolic process [GO:0042343]; is a type of indole-containing compound biosynthetic process [GO:0042435] Sources: GOC:ai